regulation of cell communication by electrical coupling [GO:0010649] (biological process) Sources: GOC:dph, GOC:kmv, GOC:tb Definition: Any process that modulates the frequency, rate or extent of cell communication via electrical coupling. Cell communication via electrical coupling is the process that mediates signaling interactions between one cell and another cell by transfer of current between their adjacent cytoplasms via intercellular protein channels. Relationships: is a type of regulation of cell communication [GO:0010646]; regulates cell communication by electrical coupling [GO:0010644] Subtypes: positive regulation of cell communication by electrical coupling [GO:0010650], negative regulation of cell communication by electrical coupling [GO:0010651], regulation of cell communication by electrical coupling involved in cardiac conduction [GO:1901844]